{
  "term_label": "ciliary basal body",
  "term_id": "GO:0036064",
  "gene_symbol": "FBF1",
  "gene": "UniProtKB:Q8TES7",
  "gene_name": "Fas-binding factor 1"
}